cellular response to abscisic acid stimulus [GO:0071215] (biological process) Sources: GOC:mah Definition: Any process that results in a change in state or activity of a cell (in terms of movement, secretion, enzyme production, gene expression, etc.) as a result of an abscisic acid stimulus. Relationships: is a type of response to abscisic acid [GO:0009737]; is a type of cellular response to hormone stimulus [GO:0032870]; is a type of GO:0071396; is a type of cellular response to alcohol [GO:0097306]